{
  "term_label": "DNA-binding transcription factor activity, RNA polymerase II-specific",
  "term_id": "GO:0000981",
  "gene_name": "Hepatic leukemia factor",
  "gene_symbol": "HLF",
  "gene": "UniProtKB:Q16534"
}